{
  "term_id": "GO:0006362",
  "gene": "UniProtKB:Q9H9Y6",
  "term_label": "transcription elongation by RNA polymerase I",
  "gene_symbol": "POLR1B",
  "gene_name": "DNA-directed RNA polymerase I subunit RPA2"
}